{
  "gene_name": "Interferon kappa",
  "term_label": "extracellular space",
  "gene": "UniProtKB:Q9P0W0",
  "term_id": "GO:0005615",
  "gene_symbol": "IFNK"
}